{
  "term_label": "Unknown biological process",
  "gene_name": "Putative golgin subfamily A member 2B",
  "gene_symbol": "GOLGA2P5",
  "term_id": "UNKNOWN:0002",
  "gene": "UniProtKB:Q9HBQ8"
}